smooth endoplasmic reticulum lumen [GO:0048238] (cellular component) Sources: GOC:jid Definition: The volume enclosed by the membranes of the smooth endoplasmic reticulum. Relationships: is a type of endoplasmic reticulum lumen [GO:0005788]; is part of GO:0005790 Also known as: SER lumen, smooth ER lumen